{
  "term_label": "Unknown molecular function",
  "gene_name": "Nucleolar protein 14",
  "term_id": "UNKNOWN:0001",
  "gene_symbol": "NOP14",
  "gene": "UniProtKB:P78316"
}